cyclohexanol dehydrogenase activity [GO:0018460] (molecular function) Also known as: cyclohexanol:NAD+ oxidoreductase activity Definition: Catalysis of the reaction: cyclohexanol + NAD+ = cyclohexanone + NADH + H+. Sources: EC:1.1.1.245 Relationships: is a type of GO:0016616